{
  "term_id": "GO:0006438",
  "gene_symbol": "VARS2",
  "gene": "UniProtKB:Q5ST30",
  "term_label": "valyl-tRNA aminoacylation",
  "gene_name": "Valine--tRNA ligase, mitochondrial"
}